{
  "gene": "UniProtKB:Q9P2H3",
  "gene_name": "Intraflagellar transport protein 80 homolog",
  "term_label": "cilium",
  "gene_symbol": "IFT80",
  "term_id": "GO:0005929"
}